positive regulation of ribosomal subunit export from nucleus [GO:2000202] (biological process) Sources: GOC:mah Definition: Any process that activates or increases the frequency, rate or extent of ribosomal subunit export from nucleus. Relationships: is a type of GO:0046824; is a type of positive regulation of ribonucleoprotein complex localization [GO:2000199]; is a type of GO:2000200; positively regulates ribosomal subunit export from nucleus [GO:0000054] Also known as: positive regulation of ribosomal subunit export from cell nucleus, positive regulation of ribosomal subunit export out of nucleus, positive regulation of ribosomal subunit transport from nucleus to cytoplasm, positive regulation of ribosomal subunit-nucleus export, positive regulation of ribosome export from nucleus Subtypes: positive regulation of ribosomal large subunit export from nucleus [GO:2000205], positive regulation of ribosomal small subunit export from nucleus [GO:2000208]